positive regulation of heart looping [GO:1901209] (biological process) Also known as: activation of cardiac looping, positive regulation of cardiac looping, up regulation of cardiac looping, up regulation of heart looping, up-regulation of cardiac looping, up-regulation of heart looping, upregulation of cardiac looping, upregulation of heart looping, activation of heart looping Relationships: is a type of regulation of heart looping [GO:1901207]; is a type of GO:1905332; RO_0002213 GO:0001947 Sources: GOC:BHF, GOC:TermGenie Definition: Any process that activates or increases the frequency, rate or extent of heart looping.